{
  "gene_symbol": "DCTN6",
  "term_id": "GO:0005869",
  "term_label": "dynactin complex",
  "gene_name": "Dynactin subunit 6",
  "gene": "UniProtKB:O00399"
}